{
  "term_id": "UNKNOWN:0003",
  "gene_name": "Coiled-coil domain-containing protein 9B",
  "term_label": "Unknown cellular component",
  "gene": "UniProtKB:Q6ZUT6",
  "gene_symbol": "CCDC9B"
}